{
  "gene_name": "Protein Atg16l2",
  "term_id": "UNKNOWN:0002",
  "gene_symbol": "ATG16L2",
  "gene": "UniProtKB:Q8NAA4",
  "term_label": "Unknown biological process"
}